{
  "term_label": "cytosol",
  "gene": "UniProtKB:P34932",
  "term_id": "GO:0005829",
  "gene_name": "Heat shock 70 kDa protein 4",
  "gene_symbol": "HSPA4"
}